regulation of D-glucose import [GO:0046324] (biological process) Sources: GOC:ai Relationships: is a type of regulation of D-glucose transmembrane transport [GO:0010827]; regulates D-glucose import [GO:0046323] Definition: Any process that modulates the frequency, rate or extent of the import of the hexose monosaccharide glucose into a cell or organelle. Subtypes: GO:0046325, GO:0046326 Also known as: regulation of glucose import, regulation of glucose uptake